{
  "gene_name": "Luc7-like protein 3",
  "gene_symbol": "LUC7L3",
  "term_id": "GO:0005685",
  "gene": "UniProtKB:O95232",
  "term_label": "U1 snRNP"
}